GMP salvage [GO:0032263] (biological process) Definition: Any process which produces guanosine monophosphate from derivatives of it, without de novo synthesis. Relationships: is_a GMP biosynthetic process [GO:0006177]; is a type of purine ribonucleotide salvage [GO:0106380] Sources: GOC:mah